{
  "gene_symbol": "ELOF1",
  "term_id": "GO:0006368",
  "term_label": "transcription elongation by RNA polymerase II",
  "gene_name": "Transcription elongation factor 1 homolog",
  "gene": "UniProtKB:P60002"
}